esophagus smooth muscle contraction [GO:0014846] (biological process) Also known as: oesophagus smooth muscle contraction Sources: GOC:ef, GOC:mtg_muscle, MA:0001573, MSH:D041742 Definition: A process in which force is generated within smooth muscle tissue, resulting in a change in muscle geometry. This process occurs in the esophagus. Force generation involves a chemo-mechanical energy conversion step that is carried out by the actin/myosin complex activity, which generates force through ATP hydrolysis. The esophagus is the muscular membranous segment between the pharynx and the stomach in the upper gastrointestinal tract. Relationships: is a type of gastro-intestinal system smooth muscle contraction [GO:0014831]